{
  "gene_symbol": "CDS2",
  "term_label": "phosphatidate cytidylyltransferase activity",
  "term_id": "GO:0004605",
  "gene": "UniProtKB:O95674",
  "gene_name": "Phosphatidate cytidylyltransferase 2"
}